mRNA CDS binding [GO:1990715] (molecular function) References: PMID:25805859 Sources: GOC:kmv, SO:0000316 Also known as: mRNA coding region binding, mRNA coding sequence binding Definition: Binding to an mRNA molecule coding sequence (CDS). Relationships: is a type of GO:0003729